{
  "gene": "UniProtKB:P61313",
  "gene_symbol": "RPL15",
  "term_id": "GO:0003723",
  "gene_name": "Large ribosomal subunit protein eL15",
  "term_label": "RNA binding"
}